phosphoenolpyruvate:phosphate antiporter activity [GO:0015121] (molecular function) Sources: GOC:bf, GOC:jl Also known as: PPT, phosphoenolpyruvate/phosphate translocator Relationships: is a type of organophosphate:phosphate antiporter activity [GO:0015315]; is a type of secondary active monocarboxylate transmembrane transporter activity [GO:0015355]; is a type of phosphoenolpyruvate transmembrane transporter activity [GO:0089721] Definition: Enables the transfer of a solute or solutes from one side of a membrane to the other according to the reaction: phosphoenolpyruvate(out) + phosphate(in) = phosphoenolpyruvate(in) + phosphate(out).